formylglycine-generating oxidase activity [GO:0120147] (molecular function) Relationships: is a type of oxidoreductase activity, acting on a sulfur group of donors, oxygen as acceptor [GO:0016670] Definition: Catalysis of the reaction: A [sulfatase]-L-cysteine + O2 + 2 a thiol = a [sulfatase]-3-oxo-L-alanine + hydrogen sulfide + a disulfide + H2O. Sources: EC:1.8.3.7, RHEA:51152